{
  "gene_symbol": "AURKC",
  "term_id": "GO:0005813",
  "gene_name": "Aurora kinase C",
  "gene": "UniProtKB:Q9UQB9",
  "term_label": "centrosome"
}